N(omega),N(omega)-dimethyl-L-arginine catabolic process [GO:2001299] (biological process) Definition: The chemical reactions and pathways resulting in the breakdown of N(omega),N(omega)-dimethyl-L-arginine, a methyl-L-arginine having two methyl groups both attached to the primary amino moiety of the guanidino group. Also known as: N(omega),N(omega)-dimethyl-L-arginine breakdown, N(omega),N(omega)-dimethyl-L-arginine catabolism, N(omega),N(omega)-dimethyl-L-arginine degradation Relationships: is a type of modified amino acid catabolic process [GO:0042219]; is a type of GO:0170035; is a type of GO:0170044 References: PMID:10510241 Sources: GOC:rs